{
  "gene_symbol": "TAF8",
  "term_id": "GO:0005669",
  "gene": "UniProtKB:Q7Z7C8",
  "term_label": "transcription factor TFIID complex",
  "gene_name": "Transcription initiation factor TFIID subunit 8"
}